{
  "gene": "UniProtKB:Q8N4F7",
  "term_id": "GO:0061630",
  "gene_symbol": "RNF175",
  "gene_name": "RING finger protein 175",
  "term_label": "ubiquitin protein ligase activity"
}